{
  "gene_name": "Sortilin",
  "term_label": "Golgi to endosome transport",
  "gene": "UniProtKB:Q99523",
  "term_id": "GO:0006895",
  "gene_symbol": "SORT1"
}